{
  "gene": "UniProtKB:Q6IC98",
  "gene_symbol": "GRAMD4",
  "term_id": "GO:0034164",
  "gene_name": "GRAM domain-containing protein 4",
  "term_label": "negative regulation of toll-like receptor 9 signaling pathway"
}